{
  "gene": "UniProtKB:A0A1W2PR80",
  "gene_symbol": "A0A1W2PR80",
  "term_id": "UNKNOWN:0003",
  "gene_name": "POM121-like protein 1",
  "term_label": "Unknown cellular component"
}